{
  "term_id": "UNKNOWN:0001",
  "term_label": "Unknown molecular function",
  "gene": "UniProtKB:Q9UEU5",
  "gene_name": "G antigen 2D",
  "gene_symbol": "GAGE8"
}